{
  "gene": "UniProtKB:Q9HAU0",
  "term_label": "phosphatidylinositol-4-phosphate binding",
  "term_id": "GO:0070273",
  "gene_name": "Pleckstrin homology domain-containing family A member 5",
  "gene_symbol": "PLEKHA5"
}